sinoatrial node cell differentiation [GO:0060921] (biological process) Relationships: is a type of GO:0060920; is part of sinoatrial node development [GO:0003163] Sources: GOC:mtg_heart Also known as: SA node cell differentiation, SAN cell differentiation, sinus node cell differentiation Definition: The process in which a relatively unspecialized cell acquires specialized features of a sinoatrial (SA) node cell. SA node cells are pacemaker cells that are found in the sinoatrial node.